{
  "gene_symbol": "SCGB2A1",
  "term_id": "UNKNOWN:0001",
  "gene": "UniProtKB:O75556",
  "gene_name": "Mammaglobin-B",
  "term_label": "Unknown molecular function"
}